{
  "gene_symbol": "EXOSC3",
  "term_id": "GO:0000467",
  "gene": "UniProtKB:Q9NQT5",
  "gene_name": "Exosome complex component RRP40",
  "term_label": "exonucleolytic trimming to generate mature 3'-end of 5.8S rRNA from tricistronic rRNA transcript (SSU-rRNA, 5.8S rRNA, LSU-rRNA)"
}